negative regulation of phospholipase C/protein kinase C signal transduction [GO:0160195] (BP) Relationships: is a type of negative regulation of intracellular signal transduction [GO:1902532]; negatively regulates phospholipase C/protein kinase C signal transduction [GO:0141212] Also known as: negative regulation of PLC/PKC signal transduction References: PMID:32033984 Definition: Any process that stops, prevents or reduces the frequency, rate or extent of phospholipase C/protein kinase C signal transduction.